{
  "gene_symbol": "ZFYVE9",
  "term_id": "GO:0007179",
  "gene": "UniProtKB:O95405",
  "gene_name": "Zinc finger FYVE domain-containing protein 9",
  "term_label": "transforming growth factor beta receptor signaling pathway"
}